{
  "gene_symbol": "UCN",
  "term_label": "Unknown cellular component",
  "term_id": "UNKNOWN:0003",
  "gene": "UniProtKB:P55089",
  "gene_name": "Urocortin"
}